{
  "gene_symbol": "MAL2",
  "gene": "UniProtKB:Q969L2",
  "term_label": "myelination",
  "term_id": "GO:0042552",
  "gene_name": "Protein MAL2"
}